{
  "term_id": "GO:0044027",
  "term_label": "negative regulation of gene expression via chromosomal CpG island methylation",
  "gene": "UniProtKB:Q96PU4",
  "gene_symbol": "UHRF2",
  "gene_name": "E3 ubiquitin-protein ligase UHRF2"
}